{
  "gene_name": "MAGUK p55 subfamily member 3",
  "gene_symbol": "MPP3",
  "term_label": "plasma membrane",
  "term_id": "GO:0005886",
  "gene": "UniProtKB:Q13368"
}